{
  "gene_name": "DNA-directed RNA polymerase I subunit RPA1",
  "gene": "UniProtKB:O95602",
  "gene_symbol": "POLR1A",
  "term_label": "Unknown molecular function",
  "term_id": "UNKNOWN:0001"
}